{
  "gene_name": "Zinc finger protein 398",
  "gene": "UniProtKB:Q8TD17",
  "term_id": "GO:0006357",
  "gene_symbol": "ZNF398",
  "term_label": "regulation of transcription by RNA polymerase II"
}